{
  "gene": "UniProtKB:Q5R3I4",
  "term_label": "Unknown biological process",
  "gene_symbol": "TTC38",
  "term_id": "UNKNOWN:0002",
  "gene_name": "Tetratricopeptide repeat protein 38"
}